{
  "term_label": "transcription coactivator activity",
  "term_id": "GO:0003713",
  "gene_name": "Metastasis-associated protein MTA1",
  "gene_symbol": "MTA1",
  "gene": "UniProtKB:Q13330"
}